{
  "term_label": "cristae formation",
  "gene_name": "MICOS complex subunit MIC13",
  "term_id": "GO:0042407",
  "gene_symbol": "MICOS13",
  "gene": "UniProtKB:Q5XKP0"
}